{
  "gene": "UniProtKB:O75251",
  "term_id": "GO:0015990",
  "gene_symbol": "NDUFS7",
  "gene_name": "NADH dehydrogenase [ubiquinone] iron-sulfur protein 7, mitochondrial",
  "term_label": "electron transport coupled proton transport"
}